{
  "term_label": "phosphotransferase activity, alcohol group as acceptor",
  "gene_name": "Glycosaminoglycan xylosylkinase",
  "gene_symbol": "FAM20B",
  "gene": "UniProtKB:O75063",
  "term_id": "GO:0016773"
}